L-ornithine catabolic process via proline [GO:0019466] (biological process) Relationships: is_a GO:0006560; is a type of L-ornithine catabolic process [GO:0006593] Sources: GOC:go_curators Also known as: ornithine breakdown via proline, ornithine degradation via proline Definition: The chemical reactions and pathways resulting in the breakdown of L-ornithine, via the intermediate proline.